regulation of plant-type cell wall organization or biogenesis [GO:0080157] (BP) References: PMID:20530756 Relationships: is a type of regulation of cell wall organization or biogenesis [GO:1903338]; regulates plant-type cell wall organization or biogenesis [GO:0071669] Also known as: regulation of plant-type cell wall organisation or biogenesis Definition: Any process that modulates the frequency, rate or extent of the chemical reactions and pathways involving plant-type cell wall organization or biogenesis. Plant-type cell wall organization or biogenesis is a process that results in the biosynthesis of constituent macromolecules, assembly, arrangement of constituent parts, or disassembly of a cellulose- and pectin-containing cell wall.